{
  "term_id": "GO:0004407",
  "term_label": "histone deacetylase activity",
  "gene_name": "Histone deacetylase 9",
  "gene": "UniProtKB:Q9UKV0",
  "gene_symbol": "HDAC9"
}